{
  "gene": "UniProtKB:Q96KN3",
  "term_label": "RNA polymerase II cis-regulatory region sequence-specific DNA binding",
  "gene_symbol": "PKNOX2",
  "term_id": "GO:0000978",
  "gene_name": "Homeobox protein PKNOX2"
}